{
  "gene_name": "Class A basic helix-loop-helix protein 9",
  "term_id": "GO:0000977",
  "gene_symbol": "BHLHA9",
  "term_label": "RNA polymerase II transcription regulatory region sequence-specific DNA binding",
  "gene": "UniProtKB:Q7RTU4"
}